{
  "term_label": "cilium organization",
  "gene_name": "Centrosomal protein of 78 kDa",
  "term_id": "GO:0044782",
  "gene_symbol": "CEP78",
  "gene": "UniProtKB:Q5JTW2"
}